{
  "gene": "UniProtKB:Q8TCE9",
  "gene_symbol": "LGALS14",
  "term_label": "Unknown cellular component",
  "term_id": "UNKNOWN:0003",
  "gene_name": "Placental protein 13-like"
}